{
  "gene": "UniProtKB:P24530",
  "gene_name": "Endothelin receptor type B",
  "gene_symbol": "EDNRB",
  "term_label": "plasma membrane",
  "term_id": "GO:0005886"
}